{
  "gene_symbol": "MYBBP1A",
  "gene_name": "Myb-binding protein 1A",
  "gene": "UniProtKB:Q9BQG0",
  "term_label": "transcription corepressor activity",
  "term_id": "GO:0003714"
}